vesicle fusion to plasma membrane [GO:0099500] (biological process) Definition: Fusion of the membrane of a vesicle with the plasma membrane, thereby releasing its contents into the extracellular space. References: PMID:18618940 Sources: GOC:aruk, GOC:bc, ISBN:0071120009 Subtypes: synaptic vesicle fusion to presynaptic active zone membrane [GO:0031629], multivesicular body fusion to apical plasma membrane [GO:0098866] Relationships: is a type of vesicle fusion [GO:0006906]; is a type of exocytic process [GO:0140029]